{
  "term_id": "GO:0009897",
  "term_label": "external side of plasma membrane",
  "gene_name": "Tumor necrosis factor receptor superfamily member 14",
  "gene": "UniProtKB:Q92956",
  "gene_symbol": "TNFRSF14"
}